{
  "term_id": "GO:0005634",
  "gene": "UniProtKB:P09960",
  "term_label": "nucleus",
  "gene_name": "Leukotriene A-4 hydrolase",
  "gene_symbol": "LTA4H"
}